photosystem stoichiometry adjustment [GO:0080005] (biological process) References: PMID:11607105 Definition: Adjustment of Photosystem I/Photosystem II ratio in response to light conditions. The function of photosystem stoichiometry adjustment is to compensate for any deficiency in energy conversion at either photosystem I or photosystem II by increasing the quantity the photosystem that will otherwise become the rate-limiting to overall photosynthesis. Relationships: is a type of GO:0010109